{
  "term_id": "GO:0043495",
  "term_label": "protein-membrane adaptor activity",
  "gene": "UniProtKB:Q2TAZ0",
  "gene_name": "Autophagy-related protein 2 homolog A",
  "gene_symbol": "ATG2A"
}